{
  "gene_name": "Zinc finger protein 217",
  "gene_symbol": "ZNF217",
  "term_id": "GO:0006355",
  "gene": "UniProtKB:O75362",
  "term_label": "regulation of DNA-templated transcription"
}